{
  "term_id": "GO:0005829",
  "gene": "UniProtKB:Q8NHS2",
  "term_label": "cytosol",
  "gene_symbol": "GOT1L1",
  "gene_name": "Putative aspartate aminotransferase, cytoplasmic 2"
}